{
  "gene": "UniProtKB:A6NEC2",
  "term_id": "GO:0005576",
  "gene_symbol": "NPEPPSL1",
  "term_label": "extracellular region",
  "gene_name": "Puromycin-sensitive aminopeptidase-like protein"
}